halogenated hydrocarbon metabolic process [GO:0042197] (biological process) Subtypes: 4-chlorobiphenyl metabolic process [GO:0018880], carbon tetrachloride metabolic process [GO:0018885], dichloromethane metabolic process [GO:0018900], 1,3-dichloropropene metabolic process [GO:0018903], methyl fluoride metabolic process [GO:0018929], GO:0018976, 1,1,1-trichloro-2,2-bis-(4-chlorophenyl)ethane metabolic process [GO:0018977], trichloroethylene metabolic process [GO:0018979], GO:0019497, halogenated hydrocarbon catabolic process [GO:0042206] Sources: GOC:ai, GOC:krc Also known as: halogenated hydrocarbon metabolism Definition: The chemical reactions and pathways involving halogenated hydrocarbons, compounds derived from hydrocarbons by replacing one or more hydrogen atoms with halogen atoms. Halogens include fluorine, chlorine, bromine and iodine. Relationships: is a type of GO:0006805; is a type of GO:0090345